{
  "term_label": "plasma membrane",
  "gene_name": "Repulsive guidance molecule A",
  "term_id": "GO:0005886",
  "gene_symbol": "RGMA",
  "gene": "UniProtKB:Q96B86"
}